benzyl isoquinoline alkaloid biosynthetic process [GO:0009708] (biological process) Definition: The chemical reactions and pathways resulting in the formation of benzyl isoquinoline alkaloids, compounds with bicyclic N-containing aromatic rings. Sources: GOC:ai, ISBN:0198506732 Also known as: benzyl isoquinoline alkaloid anabolism, benzyl isoquinoline alkaloid biosynthesis, benzyl isoquinoline alkaloid formation, benzyl isoquinoline alkaloid synthesis Subtypes: berbamunine biosynthetic process [GO:0035833], (S)-reticuline biosynthetic process [GO:1901012] Relationships: is a type of GO:0033075